{
  "gene_symbol": "DNHD1",
  "term_label": "minus-end-directed microtubule motor activity",
  "gene": "UniProtKB:Q96M86",
  "gene_name": "Dynein heavy chain domain-containing protein 1",
  "term_id": "GO:0008569"
}